regulation of glutamate receptor clustering [GO:0106104] (BP) Relationships: is a type of regulation of receptor clustering [GO:1903909]; regulates glutamate receptor clustering [GO:0097688] References: PMID:28455372 Sources: GOC:ha Definition: Any process that modulates the frequency, rate or extent of glutamate receptor clustering. Subtypes: regulation of AMPA glutamate receptor clustering [GO:1904717]